positive regulation of protein depolymerization [GO:1901881] (biological process) Relationships: is a type of positive regulation of protein-containing complex disassembly [GO:0043243]; is a type of regulation of protein depolymerization [GO:1901879]; RO_0002213 protein depolymerization [GO:0051261] References: PMID:12032137 Sources: GOC:BHF, GOC:TermGenie, GOC:rl Subtypes: GO:0030836, positive regulation of intermediate filament depolymerization [GO:0030844], positive regulation of microtubule depolymerization [GO:0031117], GO:1903390 Also known as: activation of protein polymer breakdown, activation of protein polymer catabolic process, activation of protein polymer catabolism, activation of protein polymer degradation, positive regulation of protein polymer breakdown, positive regulation of protein polymer catabolic process, positive regulation of protein polymer catabolism, positive regulation of protein polymer degradation, up regulation of protein depolymerization, up regulation of protein polymer breakdown, up regulation of protein polymer catabolic process, up regulation of protein polymer catabolism, up regulation of protein polymer degradation, up-regulation of protein depolymerization, up-regulation of protein polymer breakdown, up-regulation of protein polymer catabolic process, up-regulation of protein polymer catabolism, up-regulation of protein polymer degradation, upregulation of protein depolymerization, upregulation of protein polymer breakdown, upregulation of protein polymer catabolic process, upregulation of protein polymer catabolism, upregulation of protein polymer degradation, activation of protein depolymerization Definition: Any process that activates or increases the frequency, rate or extent of protein depolymerization.